{
  "gene": "UniProtKB:Q70J99",
  "gene_name": "Protein unc-13 homolog D",
  "gene_symbol": "UNC13D",
  "term_label": "Unknown molecular function",
  "term_id": "UNKNOWN:0001"
}